{
  "term_label": "spindle pole",
  "gene_name": "Cytoplasmic dynein 2 intermediate chain 1",
  "gene_symbol": "DYNC2I1",
  "term_id": "GO:0000922",
  "gene": "UniProtKB:Q8WVS4"
}